{
  "gene_symbol": "MXRA7",
  "term_label": "Unknown cellular component",
  "gene": "UniProtKB:P84157",
  "gene_name": "Matrix-remodeling-associated protein 7",
  "term_id": "UNKNOWN:0003"
}